{
  "term_id": "GO:0043197",
  "gene": "UniProtKB:Q9BYB0",
  "term_label": "dendritic spine",
  "gene_symbol": "SHANK3",
  "gene_name": "SH3 and multiple ankyrin repeat domains protein 3"
}